{
  "gene": "UniProtKB:Q9Y5K6",
  "term_label": "cell leading edge",
  "term_id": "GO:0031252",
  "gene_name": "CD2-associated protein",
  "gene_symbol": "CD2AP"
}